{
  "gene": "UniProtKB:A0A8V8TNH8",
  "term_id": "UNKNOWN:0003",
  "gene_symbol": "FAM90A11P",
  "gene_name": "Family with sequence similarity 90 member A11, pseudogene",
  "term_label": "Unknown cellular component"
}